{
  "gene": "UniProtKB:Q6P2H8",
  "gene_name": "Transmembrane protein 53",
  "term_id": "UNKNOWN:0001",
  "gene_symbol": "TMEM53",
  "term_label": "Unknown molecular function"
}